S-glycoside biosynthetic process [GO:0016144] (biological process) Subtypes: glucosinolate biosynthetic process [GO:0019761], lincomycin biosynthetic process [GO:1901774] Also known as: S-glycoside anabolism, S-glycoside biosynthesis, S-glycoside formation, S-glycoside synthesis, thioglycoside biosynthesis, thioglycoside biosynthetic process Definition: The chemical reactions and pathways resulting in the formation of S-glycosides, any compound in which a glycosyl group has been substituted into a thiol group. Sources: ISBN:0198506732 Relationships: is a type of sulfur compound biosynthetic process [GO:0044272]; is a type of glycosyl compound biosynthetic process [GO:1901659]